{
  "term_label": "transcription factor TFIIH holo complex",
  "term_id": "GO:0005675",
  "gene_name": "General transcription factor IIH subunit 4",
  "gene_symbol": "GTF2H4",
  "gene": "UniProtKB:Q92759"
}